{
  "term_id": "GO:0005102",
  "gene": "UniProtKB:P06239",
  "gene_symbol": "LCK",
  "gene_name": "Tyrosine-protein kinase Lck",
  "term_label": "signaling receptor binding"
}